{
  "gene_name": "Small acidic protein",
  "gene": "UniProtKB:O00193",
  "term_label": "Unknown molecular function",
  "gene_symbol": "SMAP",
  "term_id": "UNKNOWN:0001"
}